{
  "gene": "UniProtKB:O60711",
  "term_label": "focal adhesion",
  "gene_symbol": "LPXN",
  "term_id": "GO:0005925",
  "gene_name": "Leupaxin"
}